positive regulation of viral genome replication [GO:0045070] (BP) Subtypes: positive regulation of single stranded viral RNA replication via double stranded DNA intermediate [GO:0045870] Sources: GOC:ai Relationships: is_a regulation of viral genome replication [GO:0045069]; is a type of positive regulation of viral process [GO:0048524]; positively regulates viral genome replication [GO:0019079] Definition: Any process that activates or increases the frequency, rate or extent of viral genome replication. Also known as: up regulation of viral genome replication, up-regulation of viral genome replication, upregulation of viral genome replication, activation of viral genome replication, stimulation of viral genome replication